{
  "term_id": "UNKNOWN:0003",
  "gene_symbol": "KRTAP8-1",
  "term_label": "Unknown cellular component",
  "gene": "UniProtKB:Q8IUC2",
  "gene_name": "Keratin-associated protein 8-1"
}